{
  "gene": "UniProtKB:O95445",
  "term_id": "GO:0034380",
  "term_label": "high-density lipoprotein particle assembly",
  "gene_name": "Apolipoprotein M",
  "gene_symbol": "APOM"
}